{
  "term_id": "GO:0003834",
  "term_label": "beta-carotene 15,15'-dioxygenase activity",
  "gene": "UniProtKB:Q9BYV7",
  "gene_symbol": "BCO2",
  "gene_name": "Carotenoid-cleaving dioxygenase, mitochondrial"
}